procollagen-proline 4-dioxygenase complex [GO:0016222] (cellular component) Subtypes: procollagen-proline 4-dioxygenase complex, alpha(I) type [GO:0070386], procollagen-proline 4-dioxygenase complex, alpha(II) type [GO:0070387], GO:0070388 Also known as: prolyl 4-hydroxylase complex, procollagen-proline, 2-oxoglutarate-4-dioxygenase complex Definition: A protein complex that catalyzes the formation of procollagen trans-4-hydroxy-L-proline and succinate from procollagen L-proline and 2-oxoglutarate, requiring Fe2+ and ascorbate. Contains two alpha subunits that contribute to most parts of the catalytic sites, and two beta subunits that are identical to protein-disulfide isomerase. Relationships: is a type of endoplasmic reticulum protein-containing complex [GO:0140534]; is a type of oxidoreductase complex [GO:1990204] References: PMID:14500733, PMID:7753822